{
  "gene_symbol": "ATCAY",
  "term_id": "GO:0005737",
  "term_label": "cytoplasm",
  "gene_name": "Caytaxin",
  "gene": "UniProtKB:Q86WG3"
}